{
  "gene_name": "Ileal sodium_bile acid cotransporter",
  "term_id": "GO:0015721",
  "term_label": "bile acid and bile salt transport",
  "gene": "UniProtKB:Q12908",
  "gene_symbol": "SLC10A2"
}